specification of sepal identity [GO:0010096] (biological process) Relationships: is a type of specification of floral organ identity [GO:0010093]; is part of sepal formation [GO:0048453] Sources: GOC:tair_curators Definition: The process in which a floral organ primordium acquires sepal identity. Identity is considered to be the aggregate of characteristics by which a structure is recognized.